positive regulation of compound eye photoreceptor cell differentiation [GO:0110117] (biological process) References: PMID:16377567 Sources: GOC:ha Subtypes: positive regulation of R7 cell differentiation [GO:0045678], positive regulation of R8 cell differentiation [GO:0045681] Definition: Any process that activates or increases the frequency, rate or extent of compound eye photoreceptor cell differentiation. Relationships: is a type of GO:0046534; is a type of regulation of compound eye photoreceptor cell differentiation [GO:0110116]; positively regulates compound eye photoreceptor cell differentiation [GO:0001751]